{
  "term_label": "endoplasmic reticulum lumen",
  "term_id": "GO:0005788",
  "gene_name": "Protein OS-9",
  "gene": "UniProtKB:Q13438",
  "gene_symbol": "OS9"
}